{
  "gene_name": "A disintegrin and metalloproteinase with thrombospondin motifs 17",
  "gene_symbol": "ADAMTS17",
  "term_id": "GO:0004222",
  "gene": "UniProtKB:Q8TE56",
  "term_label": "metalloendopeptidase activity"
}